mycothiol synthase activity [GO:0035447] (molecular function) References: PMID:12033919 Sources: EC:2.3.1.189 Also known as: acetyl-CoA:Cys-GlcN-Ins acetyltransferase Definition: Catalysis of the reaction: 1D-myo-inositol-2-(L-cysteinylamido)-2-deoxy-alpha-D-glucopyranoside + acetyl-CoA = mycothiol + coA + H+. Mycothiol is also known as AcCys-GlcN-Ins and 1-D-myo-inosityl-2-L-cysteinylamido-2-deoxy-alpha-D-glucopyranoside as Cys-GlcN-Ins or desacetylmycothiol. Relationships: is a type of acyltransferase activity, transferring groups other than amino-acyl groups [GO:0016747]